{
  "term_label": "synapse",
  "gene_symbol": "C1QL2",
  "term_id": "GO:0045202",
  "gene": "UniProtKB:Q7Z5L3",
  "gene_name": "Complement C1q-like protein 2"
}